longitudinal flagellum [GO:0097609] (cellular component) Sources: GOC:at, Wikipedia:Dinoflagellate#Morphology, http://tolweb.org/Dinoflagellates/2445, https://doi.org/10.1508/cytologia.88.321 Also known as: longitudinal cilium Relationships: is a type of 9+2 motile cilium [GO:0097729] Definition: A motile cilium found in dinoflagellates. It trails the cell and acts as a steering rudder. It is often partially contained in a furrow called the sulcus, and emerges from a flagellar pore located in the sulcus. Note: Note that we deem cilium and microtubule-based flagellum to be equivalent. In this case community usage refers to 'flagellum' rather than 'cilium', hence the primary term name, but the cilium parentage is deliberate.